{
  "gene_symbol": "PLA2G4A",
  "term_id": "GO:0005544",
  "gene_name": "Cytosolic phospholipase A2",
  "term_label": "calcium-dependent phospholipid binding",
  "gene": "UniProtKB:P47712"
}